{
  "term_id": "GO:0005615",
  "gene_name": "Uteroglobin",
  "gene": "UniProtKB:P11684",
  "term_label": "extracellular space",
  "gene_symbol": "SCGB1A1"
}